{
  "term_label": "cGMP biosynthetic process",
  "gene_name": "Natriuretic peptides B",
  "term_id": "GO:0006182",
  "gene": "UniProtKB:P16860",
  "gene_symbol": "NPPB"
}